response to diuretic [GO:0036270] (biological process) Relationships: is a type of response to chemical [GO:0042221] Definition: Any process that results in a change in state or activity of a cell or an organism (in terms of movement, secretion, enzyme production, gene expression, etc.) as a result of a diuretic stimulus. A diuretic is an agent that promotes the excretion of urine through its effects on kidney function. Sources: GOC:hp Note: Note that this term is in the subset of terms that should not be used for direct manual annotation of gene products. It was created to be used for cross-referencing by other ontologies. Direct annotations to this term may be amended during annotation QC.